{
  "gene_name": "Insulin-like growth factor-binding protein 5",
  "gene": "UniProtKB:P24593",
  "term_id": "GO:0031995",
  "term_label": "insulin-like growth factor II binding",
  "gene_symbol": "IGFBP5"
}